{
  "gene_symbol": "PPP1R15B",
  "term_id": "GO:0000164",
  "gene_name": "Protein phosphatase 1 regulatory subunit 15B",
  "term_label": "protein phosphatase type 1 complex",
  "gene": "UniProtKB:Q5SWA1"
}